{
  "term_label": "7-dehydrocholesterol reductase activity",
  "gene": "UniProtKB:Q9UBM7",
  "term_id": "GO:0047598",
  "gene_name": "7-dehydrocholesterol reductase",
  "gene_symbol": "DHCR7"
}